CDP-diacylglycerol catabolic process [GO:0046342] (biological process) Relationships: is a type of CDP-diacylglycerol metabolic process [GO:0046341]; is a type of glycerophospholipid catabolic process [GO:0046475] Also known as: CDP-diacylglycerol breakdown, CDP-diacylglycerol catabolism, CDP-diacylglycerol degradation References: PMID:6147353 Definition: The chemical reactions and pathways resulting in the breakdown of CDP-diacylglycerol, CDP-1,2-diacylglycerol, a substance composed of diacylglycerol in glycosidic linkage with cytidine diphosphate.